{
  "term_id": "GO:0004252",
  "gene_symbol": "CLPP",
  "gene": "UniProtKB:Q16740",
  "term_label": "serine-type endopeptidase activity",
  "gene_name": "ATP-dependent Clp protease proteolytic subunit, mitochondrial"
}